{
  "gene_symbol": "PABPC1L2A",
  "term_label": "cytosol",
  "gene_name": "Polyadenylate-binding protein 1-like 2",
  "gene": "UniProtKB:Q5JQF8",
  "term_id": "GO:0005829"
}